cell-matrix adhesion mediator activity [GO:0098634] (molecular function) Sources: Wikipedia:Cell_adhesion Relationships: is a type of GO:0098631; is part of cell-matrix adhesion [GO:0007160] Definition: The binding by a cell-adhesion protein on the cell surface to an extracellular matrix component, to mediate adhesion of the cell to the extracellular matrix. Subtypes: laminin binding involved in cell-matrix adhesion [GO:0098638], collagen binding involved in cell-matrix adhesion [GO:0098639], integrin binding involved in cell-matrix adhesion [GO:0098640] Also known as: cell-matrix adhesion molecule, protein binding involved in cell-matrix adhesion